{
  "term_id": "UNKNOWN:0002",
  "term_label": "Unknown biological process",
  "gene_name": "Serpin B13",
  "gene_symbol": "SERPINB13",
  "gene": "UniProtKB:Q9UIV8"
}